{
  "gene_name": "Acylpyruvase FAHD1, mitochondrial",
  "term_id": "GO:0018773",
  "term_label": "acetylpyruvate hydrolase activity",
  "gene": "UniProtKB:Q6P587",
  "gene_symbol": "FAHD1"
}